{
  "gene": "UniProtKB:Q5QNW6",
  "gene_name": "Histone H2B type 2-F",
  "term_label": "antibacterial humoral response",
  "term_id": "GO:0019731",
  "gene_symbol": "H2BC18"
}